thioredoxin peroxidase activity [GO:0008379] (molecular function) Relationships: is a type of thioredoxin-dependent peroxiredoxin activity [GO:0140824] Also known as: TPx activity, TrxPx activity, thiol peroxidase activity Sources: RHEA:63528 Definition: Catalysis of the reaction: [thioredoxin]-dithiol + hydrogen peroxide = [thioredoxin]-disulfide + H2O. Regulation: negatively regulated by negative regulation of thioredoxin peroxidase activity by peptidyl-threonine phosphorylation [GO:1903125]